regulation of rate of cell growth [GO:0061388] (biological process) Sources: GOC:mah, GOC:vw Definition: Any process that modulates the rate of cell growth. Relationships: is a type of regulation of cell growth [GO:0001558]